{
  "term_id": "GO:0005737",
  "gene_name": "Protein bicaudal C homolog 1",
  "gene_symbol": "BICC1",
  "term_label": "cytoplasm",
  "gene": "UniProtKB:Q9H694"
}